{
  "term_id": "GO:0005802",
  "term_label": "trans-Golgi network",
  "gene_symbol": "TBC1D23",
  "gene": "UniProtKB:Q9NUY8",
  "gene_name": "TBC1 domain family member 23"
}